{
  "gene": "UniProtKB:O95166",
  "term_label": "GABA receptor binding",
  "gene_name": "Gamma-aminobutyric acid receptor-associated protein",
  "term_id": "GO:0050811",
  "gene_symbol": "GABARAP"
}